{
  "gene_name": "Chromatin accessibility complex protein 1",
  "term_label": "nucleus",
  "gene_symbol": "CHRAC1",
  "gene": "UniProtKB:Q9NRG0",
  "term_id": "GO:0005634"
}